{
  "gene_symbol": "NNT",
  "term_id": "GO:0006740",
  "term_label": "NADPH regeneration",
  "gene_name": "NAD(P) transhydrogenase, mitochondrial",
  "gene": "UniProtKB:Q13423"
}